{
  "gene_symbol": "LRRN4CL",
  "term_label": "Unknown cellular component",
  "term_id": "UNKNOWN:0003",
  "gene_name": "LRRN4 C-terminal-like protein",
  "gene": "UniProtKB:Q8ND94"
}